{
  "term_id": "GO:0097250",
  "gene_name": "HIG1 domain family member 2A, mitochondrial",
  "term_label": "mitochondrial respirasome assembly",
  "gene": "UniProtKB:Q9BW72",
  "gene_symbol": "HIGD2A"
}